snoRNA release from pre-rRNA [GO:1990417] (BP) Relationships: is a type of rRNA processing [GO:0006364] References: PMID:16908538 Sources: GOC:rb Note: An example of this process is yeast HAS1 from PMID:16908538, inferred from mutant phenotype assay. Definition: The release of snoRNA from pre-rRNA.